L-glutamate transmembrane transport [GO:0015813] (biological process) Definition: The directed movement of L-glutamate across a membrane by means of some agent such as a transporter or a pore. Also known as: L-glutamate transport, mitochondrial aspartate/glutamate transport References: PMID:21307582 Subtypes: L-glutamate transmembrane export from vacuole [GO:0089704], L-glutamate transmembrane import into vacuole [GO:0090515], GO:0098712, L-glutamate import into mitochondrion [GO:0110141] Relationships: is a type of L-glutamate import [GO:0051938]; is a type of L-alpha-amino acid transmembrane transport [GO:1902475]